{
  "gene": "UniProtKB:P01566",
  "gene_name": "Interferon alpha-10",
  "term_label": "type I interferon-mediated signaling pathway",
  "term_id": "GO:0060337",
  "gene_symbol": "IFNA10"
}